alphav-beta1 integrin-osteopontin complex [GO:0070030] (cellular component) Relationships: is a type of plasma membrane protein complex [GO:0098797] Definition: A protein complex that consists of an alphav-beta1 integrin complex bound to osteopontin. References: PMID:7592829 Also known as: ITGAV-ITGB1-SPP1 complex